{
  "gene_name": "Elongation factor 1-beta",
  "term_label": "cytosol",
  "gene": "UniProtKB:P24534",
  "term_id": "GO:0005829",
  "gene_symbol": "EEF1B2"
}